{
  "gene": "UniProtKB:Q9NRX4",
  "term_id": "GO:0101006",
  "term_label": "protein histidine phosphatase activity",
  "gene_name": "14 kDa phosphohistidine phosphatase",
  "gene_symbol": "PHPT1"
}